3-phosphoglycerate phosphatase activity [GO:0047572] (MF) Definition: Catalysis of the reaction: 3-phospho-D-glycerate + H2O = D-glycerate + phosphate. Sources: EC:3.1.3.38, RHEA:12412 Also known as: 3-PGA phosphatase activity, D-3-phosphoglycerate phosphatase activity, D-glycerate-3-phosphate phosphohydrolase activity Relationships: is a type of phosphatase activity [GO:0016791]